male pronucleus [GO:0001940] (CC) Sources: GOC:hjd, ISBN:0198506732 Relationships: is a type of GO:0045120 Definition: The pronucleus originating from the spermatozoa that was involved in fertilization.